{
  "gene_name": "Mitochondrial import receptor subunit TOM40 homolog",
  "gene_symbol": "TOMM40",
  "term_label": "mitochondrial outer membrane translocase complex",
  "gene": "UniProtKB:O96008",
  "term_id": "GO:0005742"
}